{
  "term_label": "vesicle docking",
  "gene": "UniProtKB:P32856",
  "gene_symbol": "STX2",
  "term_id": "GO:0048278",
  "gene_name": "Syntaxin-2"
}